{
  "gene_name": "F-box_WD repeat-containing protein 5",
  "gene_symbol": "FBXW5",
  "term_label": "Unknown biological process",
  "term_id": "UNKNOWN:0002",
  "gene": "UniProtKB:Q969U6"
}